{
  "gene_symbol": "FKBP9P1",
  "term_label": "Unknown molecular function",
  "term_id": "UNKNOWN:0001",
  "gene": "UniProtKB:Q75LS8",
  "gene_name": "Putative FK506-binding protein 9-like protein"
}